{
  "gene_name": "Interferon alpha-17",
  "gene": "UniProtKB:P01571",
  "term_id": "GO:0005132",
  "gene_symbol": "IFNA17",
  "term_label": "type I interferon receptor binding"
}